{
  "term_id": "GO:0000981",
  "gene_symbol": "ZNF823",
  "gene_name": "Zinc finger protein 823",
  "gene": "UniProtKB:P16415",
  "term_label": "DNA-binding transcription factor activity, RNA polymerase II-specific"
}